{
  "term_label": "positive regulation of transcription by RNA polymerase II",
  "gene_name": "PAX3- and PAX7-binding protein 1",
  "gene_symbol": "PAXBP1",
  "term_id": "GO:0045944",
  "gene": "UniProtKB:Q9Y5B6"
}